{
  "gene": "UniProtKB:Q14D33",
  "term_id": "GO:0031849",
  "gene_symbol": "RTP5",
  "gene_name": "Receptor-transporting protein 5",
  "term_label": "olfactory receptor binding"
}